ecgonine methyl ester catabolic process [GO:1901868] (biological process) Also known as: ecgonine methyl ester breakdown, ecgonine methyl ester catabolism, ecgonine methyl ester degradation Definition: The chemical reactions and pathways resulting in the breakdown of ecgonine methyl ester. Relationships: is a type of GO:0009822 References: PMID:22665766 Sources: GOC:TermGenie